{
  "term_id": "GO:0005886",
  "gene_name": "Pleckstrin homology domain-containing family A member 2",
  "gene": "UniProtKB:Q9HB19",
  "gene_symbol": "PLEKHA2",
  "term_label": "plasma membrane"
}